{
  "term_label": "box C/D snoRNP assembly",
  "term_id": "GO:0000492",
  "gene_name": "FMR1-interacting protein NUFIP1",
  "gene_symbol": "NUFIP1",
  "gene": "UniProtKB:Q9UHK0"
}